adipokinetic hormone receptor activity [GO:0097003] (molecular function) Relationships: is a type of protein-hormone receptor activity [GO:0016500]; has part GO:0055100; has part adipokinetic hormone binding [GO:0097004] Definition: Combining with an adipokinetic hormone to initiate a change in cell activity. Adipokinetic hormones (AKHs) are protein or peptide hormones that are important for sugar and fat homeostasis in metazoa. In insects, they mobilize sugar and lipids from the insect fat body during energy-requiring activities such as flight and locomotion. They also contribute to hemolymph sugar homeostasis. References: PMID:11904407 Sources: GOC:sart Also known as: AKH receptor activity